{
  "gene": "UniProtKB:Q9Y3U8",
  "gene_symbol": "RPL36",
  "gene_name": "Large ribosomal subunit protein eL36",
  "term_label": "structural constituent of ribosome",
  "term_id": "GO:0003735"
}